negative regulation of potassium ion export across plasma membrane [GO:1903765] (biological process) Also known as: down regulation of potassium export, down regulation of potassium ion export, down-regulation of potassium export, down-regulation of potassium ion export, downregulation of potassium export, downregulation of potassium ion export, negative regulation of potassium export, negative regulation of potassium ion export, down regulation of potassium ion export across plasma membrane, down-regulation of potassium ion export across plasma membrane, downregulation of potassium ion export across plasma membrane, inhibition of potassium ion export across plasma membrane, inhibition of potassium export, inhibition of potassium ion export Definition: Any process that stops, prevents or reduces the frequency, rate or extent of potassium ion export across the plasma membrane. References: PMID:19646991 Sources: GOC:BHF, GOC:TermGenie, GOC:mtg_cardiac_conduct_nov11, GOC:rl, GO_REF:0000058 Relationships: is a type of negative regulation of potassium ion transmembrane transport [GO:1901380]; is a type of regulation of potassium ion export across plasma membrane [GO:1903764]; negatively regulates potassium ion export across plasma membrane [GO:0097623]